{
  "gene": "UniProtKB:Q8IUC4",
  "gene_symbol": "RHPN2",
  "term_id": "UNKNOWN:0001",
  "term_label": "Unknown molecular function",
  "gene_name": "Rhophilin-2"
}